{
  "gene_name": "PRA1 family protein 3",
  "term_id": "UNKNOWN:0001",
  "gene_symbol": "ARL6IP5",
  "term_label": "Unknown molecular function",
  "gene": "UniProtKB:O75915"
}